{
  "term_label": "lysosome",
  "gene_symbol": "SLC17A5",
  "gene": "UniProtKB:Q9NRA2",
  "term_id": "GO:0005764",
  "gene_name": "Sialin"
}